{
  "term_id": "GO:0005634",
  "gene_symbol": "HNRNPUL2",
  "gene_name": "Heterogeneous nuclear ribonucleoprotein U-like protein 2",
  "gene": "UniProtKB:Q1KMD3",
  "term_label": "nucleus"
}